negative regulation of hemocyte differentiation [GO:0045611] (biological process) Subtypes: negative regulation of lamellocyte differentiation [GO:0035204], negative regulation of crystal cell differentiation [GO:0042690], negative regulation of plasmatocyte differentiation [GO:0045614] Also known as: down regulation of hemocyte differentiation, down-regulation of hemocyte differentiation, downregulation of hemocyte differentiation, negative regulation of arthropod blood cell differentiation, inhibition of hemocyte differentiation Relationships: is a type of negative regulation of immune system process [GO:0002683]; is a type of GO:0045596; is a type of regulation of hemocyte differentiation [GO:0045610]; negatively regulates hemocyte differentiation [GO:0042386] Definition: Any process that stops, prevents, or reduces the frequency, rate or extent of hemocyte differentiation. Sources: GOC:go_curators